{
  "gene_symbol": "ALOX5",
  "gene_name": "Polyunsaturated fatty acid 5-lipoxygenase",
  "term_label": "arachidonate 5-lipoxygenase activity",
  "term_id": "GO:0004051",
  "gene": "UniProtKB:P09917"
}